{
  "term_id": "GO:0038092",
  "term_label": "nodal signaling pathway",
  "gene": "UniProtKB:P0CG37",
  "gene_name": "Cryptic protein",
  "gene_symbol": "CFC1"
}